retrograde synaptic vesicle transport [GO:0048491] (biological process) Relationships: is a type of retrograde axonal transport [GO:0008090]; is a type of GO:0099517 Definition: The directed movement of synaptic vesicle along axonal microtubules from the presynapse to the cell body. References: PMID:24762653 Sources: GOC:jid, GOC:lmg Also known as: retrograde axonal transport of synaptic vesicle